{
  "gene": "UniProtKB:Q96MS3",
  "term_id": "UNKNOWN:0001",
  "term_label": "Unknown molecular function",
  "gene_name": "Glycosyltransferase 1 domain-containing protein 1",
  "gene_symbol": "GLT1D1"
}